{
  "gene_name": "Keratin, type I cuticular Ha4",
  "gene_symbol": "KRT34",
  "term_label": "intermediate filament organization",
  "gene": "UniProtKB:O76011",
  "term_id": "GO:0045109"
}